{
  "gene_symbol": "CADM1",
  "term_id": "GO:0008037",
  "gene_name": "Cell adhesion molecule 1",
  "term_label": "cell recognition",
  "gene": "UniProtKB:Q9BY67"
}